{
  "gene_symbol": "SYNPO2",
  "gene_name": "Synaptopodin-2",
  "gene": "UniProtKB:Q9UMS6",
  "term_id": "GO:0015629",
  "term_label": "actin cytoskeleton"
}